{
  "gene_name": "Aurora kinase A",
  "term_id": "GO:0032465",
  "gene_symbol": "AURKA",
  "gene": "UniProtKB:O14965",
  "term_label": "regulation of cytokinesis"
}